{
  "term_label": "membrane",
  "term_id": "GO:0016020",
  "gene": "UniProtKB:P59535",
  "gene_symbol": "TAS2R40",
  "gene_name": "Taste receptor type 2 member 40"
}